synaptic vesicle transport along actin filament [GO:0099506] (biological process) Sources: GOC:dos Definition: The directed movement of synaptic vesicles along actin filaments within a cell, powered by molecular motors. Relationships: is a type of vesicle transport along actin filament [GO:0030050]; is a type of synaptic vesicle cytoskeletal transport [GO:0099514]